{
  "term_id": "GO:0005737",
  "gene_name": "AFG1-like ATPase",
  "gene": "UniProtKB:Q8WV93",
  "term_label": "cytoplasm",
  "gene_symbol": "AFG1L"
}